negative regulation of dendritic spine development [GO:0061000] (BP) Relationships: is a type of negative regulation of developmental process [GO:0051093]; is a type of regulation of dendritic spine development [GO:0060998]; negatively regulates GO:0060996 Subtypes: negative regulation of dendritic spine morphogenesis [GO:0061002] Sources: GOC:dph Definition: Any process that decreases the rate, frequency, or extent of dendritic spine development, the process whose specific outcome is the progression of the dendritic spine over time, from its formation to the mature structure.